{
  "term_id": "GO:0019903",
  "gene": "UniProtKB:Q96QG7",
  "term_label": "protein phosphatase binding",
  "gene_symbol": "MTMR9",
  "gene_name": "Myotubularin-related protein 9"
}